{
  "gene": "UniProtKB:Q53FZ2",
  "gene_symbol": "ACSM3",
  "term_id": "GO:0015645",
  "gene_name": "Acyl-coenzyme A synthetase ACSM3, mitochondrial",
  "term_label": "fatty acid ligase activity"
}